{
  "gene": "UniProtKB:O14493",
  "gene_symbol": "CLDN4",
  "term_id": "GO:0005923",
  "gene_name": "Claudin-4",
  "term_label": "bicellular tight junction"
}